{
  "term_label": "chloride:bicarbonate antiporter activity",
  "gene_name": "Testis anion transporter 1",
  "gene": "UniProtKB:Q96RN1",
  "term_id": "GO:0140900",
  "gene_symbol": "SLC26A8"
}